regulation of epithelial cell differentiation [GO:0030856] (BP) Sources: GOC:mah Relationships: is_a regulation of cell differentiation [GO:0045595]; is a type of GO:2000026; regulates GO:0030855 Definition: Any process that modulates the frequency, rate or extent of epithelial cell differentiation. Subtypes: negative regulation of epithelial cell differentiation [GO:0030857], positive regulation of epithelial cell differentiation [GO:0030858], regulation of polarized epithelial cell differentiation [GO:0030860], regulation of cumulus cell differentiation [GO:0045592], GO:0045601, regulation of epidermal cell differentiation [GO:0045604], GO:0061105, regulation of hepatocyte differentiation [GO:0070366], regulation of lung ciliated cell differentiation [GO:1901246], regulation of lung goblet cell differentiation [GO:1901249], regulation of odontoblast differentiation [GO:1901329], regulation of lens fiber cell differentiation [GO:1902746], regulation of intestinal epithelial cell development [GO:1905298], regulation of pancreatic A cell differentiation [GO:2000226], regulation of epithelial cell differentiation involved in kidney development [GO:2000696]